{
  "gene": "UniProtKB:Q8NBM8",
  "term_id": "UNKNOWN:0003",
  "gene_name": "Prenylcysteine oxidase-like",
  "term_label": "Unknown cellular component",
  "gene_symbol": "PCYOX1L"
}